deacetoxycephalosporin-C synthase activity [GO:0050599] (molecular function) Relationships: is_a oxidoreductase activity, acting on paired donors, with incorporation or reduction of molecular oxygen, with 2-oxoglutarate as one donor, and the other dehydrogenated [GO:0050498] Definition: Catalysis of the reaction: 2-oxoglutarate + O2 + penicillin N = CO2 + deacetoxycephalosporin C + H2O + succinate. Also known as: deacetoxycephalosporin C synthetase activity, expandase activity, DAOC synthase activity, DAOCS activity, penicillin N expandase activity, penicillin-N,2-oxoglutarate:oxygen oxidoreductase (ring-expanding) Sources: EC:1.14.20.1, RHEA:20748